{
  "gene": "UniProtKB:Q9NUY8",
  "term_label": "vesicle tethering to Golgi",
  "term_id": "GO:0099041",
  "gene_name": "TBC1 domain family member 23",
  "gene_symbol": "TBC1D23"
}